{
  "gene_symbol": "KCNAB1",
  "gene_name": "Voltage-gated potassium channel subunit beta-1",
  "gene": "UniProtKB:Q14722",
  "term_label": "regulation of potassium ion transmembrane transport",
  "term_id": "GO:1901379"
}